{
  "term_label": "Unknown molecular function",
  "gene": "UniProtKB:Q6P3W6",
  "gene_name": "Neuroblastoma breakpoint family member 10",
  "term_id": "UNKNOWN:0001",
  "gene_symbol": "NBPF10"
}